{
  "term_label": "Unknown cellular component",
  "term_id": "UNKNOWN:0003",
  "gene": "UniProtKB:Q6NV75",
  "gene_name": "Probable G-protein coupled receptor 153",
  "gene_symbol": "GPR153"
}